{
  "gene": "UniProtKB:Q9UI17",
  "term_id": "GO:0005759",
  "term_label": "mitochondrial matrix",
  "gene_name": "Dimethylglycine dehydrogenase, mitochondrial",
  "gene_symbol": "DMGDH"
}